{
  "gene_symbol": "FTH1",
  "term_id": "GO:0006826",
  "term_label": "iron ion transport",
  "gene_name": "Ferritin heavy chain",
  "gene": "UniProtKB:P02794"
}